{
  "gene": "UniProtKB:P20823",
  "gene_symbol": "HNF1A",
  "term_id": "GO:0000978",
  "term_label": "RNA polymerase II cis-regulatory region sequence-specific DNA binding",
  "gene_name": "Hepatocyte nuclear factor 1-alpha"
}